fatty acid transport [GO:0015908] (biological process) Sources: GOC:ai Relationships: is a type of GO:0006869; is a type of monocarboxylic acid transport [GO:0015718] Definition: The directed movement of fatty acids into, out of or within a cell, or between cells, by means of some agent such as a transporter or pore. Fatty acids are aliphatic monocarboxylic acids liberated from naturally occurring fats and oils by hydrolysis. Subtypes: medium-chain fatty acid transport [GO:0001579], GO:0015732, long-chain fatty acid transport [GO:0015909], short-chain fatty acid transport [GO:0015912], thromboxane transport [GO:0071717], GO:1902001 Regulation: regulated by regulation of fatty acid transport [GO:2000191]; negatively regulated by GO:2000192; positively regulated by GO:2000193